{
  "gene": "UniProtKB:Q96H22",
  "gene_name": "Centromere protein N",
  "term_id": "UNKNOWN:0001",
  "term_label": "Unknown molecular function",
  "gene_symbol": "CENPN"
}